positive regulation of cardiac myofibril assembly [GO:1905306] (biological process) Also known as: positive regulation of cardiac myofibril development, positive regulation of cardiac myofibril morphogenesis, up regulation of cardiac myofibril assembly, up regulation of cardiac myofibril development, up regulation of cardiac myofibril morphogenesis, up-regulation of cardiac myofibril assembly, up-regulation of cardiac myofibril development, up-regulation of cardiac myofibril morphogenesis, upregulation of cardiac myofibril assembly, upregulation of cardiac myofibril development, upregulation of cardiac myofibril morphogenesis, activation of cardiac myofibril assembly, activation of cardiac myofibril development, activation of cardiac myofibril morphogenesis, activation of heart myofibril assembly, positive regulation of heart myofibril assembly, up regulation of heart myofibril assembly, up-regulation of heart myofibril assembly, upregulation of heart myofibril assembly References: PMID:16151019 Sources: GOC:BHF, GOC:TermGenie, GOC:rl, GO_REF:0000058 Definition: Any process that activates or increases the frequency, rate or extent of cardiac myofibril assembly. Relationships: is a type of positive regulation of developmental process [GO:0051094]; is a type of positive regulation of cytoskeleton organization [GO:0051495]; is a type of positive regulation of organelle assembly [GO:1902117]; is a type of positive regulation of supramolecular fiber organization [GO:1902905]; is a type of regulation of cardiac myofibril assembly [GO:1905304]; positively regulates cardiac myofibril assembly [GO:0055003]